{
  "gene_name": "Protein FAM151A",
  "gene": "UniProtKB:Q8WW52",
  "term_id": "UNKNOWN:0001",
  "term_label": "Unknown molecular function",
  "gene_symbol": "FAM151A"
}